{
  "gene_symbol": "DSG3",
  "term_id": "GO:0005509",
  "term_label": "calcium ion binding",
  "gene_name": "Desmoglein-3",
  "gene": "UniProtKB:P32926"
}